{
  "term_id": "GO:0007015",
  "gene_symbol": "MYO5C",
  "gene_name": "Unconventional myosin-Vc",
  "gene": "UniProtKB:Q9NQX4",
  "term_label": "actin filament organization"
}